regulation of timing of transition from vegetative to reproductive phase [GO:0048510] (biological process) Relationships: is a type of regulation of timing of meristematic phase transition [GO:0048506] Definition: The process controlling the point in time during development when a vegetative meristem will change its identity to become an inflorescence or floral meristem, and/or the rate at which the change occurs. References: PMID:8974397 Sources: GOC:jid